caveolar macromolecular signaling complex [GO:0002095] (CC) References: PMID:16648270 Relationships: is a type of plasma membrane protein complex [GO:0098797]; is part of caveola [GO:0005901] Definition: A complex composed of proteins required for beta adrenergic receptor activation of protein kinase A. It includes the Cav 12. subunit of L-type calcium channel, protein kinase A regulatory subunit 2(PKAR2), adenyl cyclase, beta-adrenergic receptor, G-alpha-S, protein phosphatase 2A (PP2A) and caveolin 3 (CAV3). Also known as: caveolar macromolecular signalling complex